L-methionine import across plasma membrane [GO:1905544] (biological process) Definition: The directed movement of L-methionine from outside of a cell, across the plasma membrane and into the cytosol. Relationships: is a type of L-alpha-amino acid transmembrane transport [GO:1902475]; is a type of GO:1903692 References: PMID:17556368 Sources: GOC:TermGenie, GO_REF:0000075 Also known as: L-methionine import into cell Regulation: regulated by regulation of L-methionine import across plasma membrane [GO:1905624]; negatively regulated by negative regulation of L-methionine import across plasma membrane [GO:1905625]; positively regulated by positive regulation of L-methionine import across plasma membrane [GO:1905626]